{
  "term_label": "Unknown molecular function",
  "gene_symbol": "TNRC6A",
  "gene_name": "Trinucleotide repeat-containing gene 6A protein",
  "term_id": "UNKNOWN:0001",
  "gene": "UniProtKB:Q8NDV7"
}